{
  "gene": "UniProtKB:Q9NSQ0",
  "term_label": "CURI complex",
  "term_id": "GO:0032545",
  "gene_symbol": "RRP7BP",
  "gene_name": "Putative ribosomal RNA-processing protein 7 homolog B"
}